{
  "gene_name": "Twist-related protein 2",
  "gene": "UniProtKB:Q8WVJ9",
  "term_id": "GO:0032502",
  "term_label": "developmental process",
  "gene_symbol": "TWIST2"
}